{
  "term_label": "cytoplasm",
  "gene_name": "Sterile alpha motif domain-containing protein 9",
  "term_id": "GO:0005737",
  "gene": "UniProtKB:Q5K651",
  "gene_symbol": "SAMD9"
}